{
  "gene": "UniProtKB:Q8NHA4",
  "term_label": "detection of chemical stimulus involved in sensory perception of smell",
  "term_id": "GO:0050911",
  "gene_symbol": "OR2AE1",
  "gene_name": "Olfactory receptor 2AE1"
}